{
  "gene_symbol": "MED16",
  "term_id": "GO:0060261",
  "gene": "UniProtKB:Q9Y2X0",
  "gene_name": "Mediator of RNA polymerase II transcription subunit 16",
  "term_label": "positive regulation of transcription initiation by RNA polymerase II"
}